{
  "gene": "UniProtKB:Q96MT3",
  "term_label": "Unknown cellular component",
  "gene_name": "Prickle-like protein 1",
  "term_id": "UNKNOWN:0003",
  "gene_symbol": "PRICKLE1"
}